{
  "gene": "UniProtKB:Q9H999",
  "gene_name": "Pantothenate kinase 3",
  "gene_symbol": "PANK3",
  "term_id": "GO:0005634",
  "term_label": "nucleus"
}